{
  "term_id": "GO:0006814",
  "gene": "UniProtKB:Q8N695",
  "term_label": "sodium ion transport",
  "gene_symbol": "SLC5A8",
  "gene_name": "Sodium-coupled monocarboxylate transporter 1"
}